{
  "term_label": "protein insertion into membrane",
  "term_id": "GO:0051205",
  "gene": "UniProtKB:Q96DX8",
  "gene_name": "Receptor-transporting protein 4",
  "gene_symbol": "RTP4"
}